hydroxyphytanate oxidase activity [GO:0047996] (molecular function) Also known as: L-2-hydroxyphytanate:oxygen 2-oxidoreductase Definition: Catalysis of the reaction: (2S)-2-hydroxyphytanate + O2 = 2-oxophytanate + H2O2. Sources: EC:1.1.3.27, RHEA:21680 Relationships: is a type of GO:0016899